{
  "gene_symbol": "KCNK18",
  "term_id": "GO:0071805",
  "gene": "UniProtKB:Q7Z418",
  "gene_name": "Potassium channel subfamily K member 18",
  "term_label": "potassium ion transmembrane transport"
}